{
  "term_label": "cytoplasm",
  "gene": "UniProtKB:O94761",
  "gene_symbol": "RECQL4",
  "gene_name": "ATP-dependent DNA helicase Q4",
  "term_id": "GO:0005737"
}